regulation of dendrite development [GO:0050773] (biological process) Relationships: is a type of regulation of neuron projection development [GO:0010975]; is a type of regulation of developmental process [GO:0050793]; regulates GO:0016358 Definition: Any process that modulates the frequency, rate or extent of dendrite development. Sources: GOC:ai Subtypes: regulation of dendrite morphogenesis [GO:0048814], positive regulation of dendrite development [GO:1900006], GO:2000171